negative regulation of toll-like receptor signaling pathway [GO:0034122] (biological process) References: PMID:16551253, PMID:17328678 Sources: GOC:add Also known as: negative regulation of TLR signaling pathway, negative regulation of toll-like receptor signalling pathway Subtypes: negative regulation of MyD88-dependent toll-like receptor signaling pathway [GO:0034125], negative regulation of MyD88-independent toll-like receptor signaling pathway [GO:0034128], GO:2000444 Relationships: is a type of negative regulation of immune system process [GO:0002683]; is a type of negative regulation of signal transduction [GO:0009968]; is a type of regulation of toll-like receptor signaling pathway [GO:0034121]; negatively regulates GO:0002224 Definition: Any process that stops, prevents, or reduces the frequency, rate, or extent of toll-like receptor signaling pathway.